pheromone biosynthetic process [GO:0042811] (biological process) Subtypes: 4-vinylanisole biosynthetic process [GO:0160305] Relationships: is a type of hormone biosynthetic process [GO:0042446]; is a type of GO:0042810; is_a secondary metabolite biosynthetic process [GO:0044550] Also known as: pheromone anabolism, pheromone biosynthesis, pheromone formation, pheromone synthesis Sources: ISBN:0198506732 Definition: The chemical reactions and pathways resulting in the formation of pheromones, a substance that is secreted and released by an organism and detected by a second organism of the same or a closely related species, in which it causes a specific reaction, such as a definite behavioral reaction or a developmental process.